hatching gland development [GO:0048785] (BP) Relationships: is a type of gland development [GO:0048732] Definition: The process whose specific outcome is the progression of the hatching gland over time, from its formation to the mature structure. The cells of the hatching gland contain enzymes responsible for solubilization of the egg chorion, facilitating the hatching process. Sources: GOC:bf, GOC:dh, GOC:jid